{
  "gene": "UniProtKB:Q9HCT0",
  "gene_name": "Fibroblast growth factor 22",
  "term_label": "fibroblast growth factor receptor signaling pathway",
  "term_id": "GO:0008543",
  "gene_symbol": "FGF22"
}